{
  "term_label": "nucleus",
  "gene_name": "Zinc finger protein 483",
  "gene_symbol": "ZNF483",
  "term_id": "GO:0005634",
  "gene": "UniProtKB:Q8TF39"
}